iprodione metabolic process [GO:0018922] (biological process) Sources: UM-BBD_pathwayID:ipd Definition: The chemical reactions and pathways involving prodione, a colorless, odorless crystal. It is used as a dicarboximide contact fungicide to control a wide variety of crop diseases by inhibiting the germination of spores and the growth of the fungal mat (mycelium). Also known as: iprodione metabolism Relationships: is a type of benzene-containing compound metabolic process [GO:0042537]; is a type of amide metabolic process [GO:0043603]; is a type of imidazole-containing compound metabolic process [GO:0052803]; is a type of organohalogen metabolic process [GO:0090345]